{
  "term_label": "dehydroascorbic acid transport",
  "gene_symbol": "SLC2A11",
  "term_id": "GO:0070837",
  "gene_name": "Solute carrier family 2, facilitated glucose transporter member 11",
  "gene": "UniProtKB:Q9BYW1"
}